{
  "term_label": "muscle contraction",
  "gene": "UniProtKB:P28289",
  "term_id": "GO:0006936",
  "gene_name": "Tropomodulin-1",
  "gene_symbol": "TMOD1"
}